{
  "gene_symbol": "DTX2",
  "term_id": "GO:0016567",
  "term_label": "protein ubiquitination",
  "gene_name": "Probable E3 ubiquitin-protein ligase DTX2",
  "gene": "UniProtKB:Q86UW9"
}